{
  "term_label": "glutamate receptor binding",
  "term_id": "GO:0035254",
  "gene": "UniProtKB:P24588",
  "gene_symbol": "AKAP5",
  "gene_name": "A-kinase anchor protein 5"
}